{
  "term_label": "histone methyltransferase complex",
  "gene_name": "Host cell factor 1",
  "gene": "UniProtKB:P51610",
  "term_id": "GO:0035097",
  "gene_symbol": "HCFC1"
}